{
  "gene": "UniProtKB:Q96B01",
  "term_id": "GO:0003697",
  "gene_name": "RAD51-associated protein 1",
  "term_label": "single-stranded DNA binding",
  "gene_symbol": "RAD51AP1"
}